central nervous system neuron axonogenesis [GO:0021955] (biological process) Sources: GOC:cls, GOC:dgh, GOC:dph, GOC:jid, GO_REF:0000021 Definition: Generation of a long process from a neuron whose cell body resides in the central nervous system. The process carries efferent (outgoing) action potentials from the cell body towards target cells. Relationships: is a type of axonogenesis [GO:0007409]; is part of central nervous system neuron development [GO:0021954] Subtypes: central nervous system projection neuron axonogenesis [GO:0021952], central nervous system interneuron axonogenesis [GO:0021956], GO:0048894